{
  "gene": "UniProtKB:P22674",
  "gene_symbol": "CCNO",
  "term_id": "GO:0005634",
  "gene_name": "Cyclin-O",
  "term_label": "nucleus"
}